ABC-type quaternary ammonium compound transporting activity [GO:0015418] (MF) Definition: Catalysis of the reaction: ATP + H2O + quaternary ammonium(out) = ADP + H+ + phosphate + quaternary ammonium(in). Sources: GOC:pz, RHEA:11036 Relationships: is a type of quaternary ammonium group transmembrane transporter activity [GO:0015651]; is a type of GO:0140359 Subtypes: ABC-type glycine betaine transporter activity [GO:0031459] Also known as: quarternary amine transporter activity, quaternary-ammonium-compound ABC transporter, glycine betaine/proline porter activity, ATP-dependent quaternary-ammonium compound transmembrane transporting activity, ATPase-coupled quaternary ammonium compound transmembrane transporting activity, quaternary amine uptake transporter activity, quaternary-amine-transporting ATPase activity, quaternary-ammonium-compound-transporting ATPase activity